{
  "gene_symbol": "SRSF10",
  "term_label": "mRNA binding",
  "gene": "UniProtKB:O75494",
  "gene_name": "Serine_arginine-rich splicing factor 10",
  "term_id": "GO:0003729"
}